{
  "term_label": "phospholipid-hydroperoxide glutathione peroxidase activity",
  "gene_name": "Phospholipid hydroperoxide glutathione peroxidase",
  "gene_symbol": "GPX4",
  "gene": "UniProtKB:P36969",
  "term_id": "GO:0047066"
}